prolactin receptor activity [GO:0004925] (MF) Relationships: is a type of cytokine receptor activity [GO:0004896]; is part of prolactin signaling pathway [GO:0038161] Sources: GOC:mah, GOC:signaling Definition: Combining with prolactin and transmitting the signal from one side of the membrane to the other to initiate a change in cell activity.